integrin complex [GO:0008305] (CC) Relationships: is a type of GO:0098636; is a type of GO:0098802 Definition: A protein complex that is composed of one alpha subunit and one beta subunit, both of which are members of the integrin superfamily of cell adhesion receptors; the complex spans the plasma membrane and binds to extracellular matrix ligands, cell-surface ligands, and soluble ligands. Also known as: laminin receptor protein References: PMID:17543136 Subtypes: GO:0034665, integrin alpha2-beta1 complex [GO:0034666], integrin alpha3-beta1 complex [GO:0034667], GO:0034668, integrin alpha4-beta7 complex [GO:0034669], integrin alpha5-beta1 complex [GO:0034674], integrin alpha6-beta1 complex [GO:0034675], integrin alpha6-beta4 complex [GO:0034676], GO:0034677, integrin alpha8-beta1 complex [GO:0034678], integrin alpha9-beta1 complex [GO:0034679], integrin alpha10-beta1 complex [GO:0034680], integrin alpha11-beta1 complex [GO:0034681], integrin alphav-beta1 complex [GO:0034682], GO:0034683, integrin alphav-beta5 complex [GO:0034684], integrin alphav-beta6 complex [GO:0034685], integrin alphav-beta8 complex [GO:0034686], integrin alphaL-beta2 complex [GO:0034687], GO:0034688, integrin alphaX-beta2 complex [GO:0034689], GO:0034690, integrin alphaE-beta7 complex [GO:0034691], integrin alphaIIb-beta3 complex [GO:0070442]